{
  "term_id": "GO:0140658",
  "gene": "UniProtKB:Q14839",
  "gene_name": "Chromodomain-helicase-DNA-binding protein 4",
  "gene_symbol": "CHD4",
  "term_label": "ATP-dependent chromatin remodeler activity"
}